{
  "gene": "UniProtKB:O94806",
  "gene_name": "Serine_threonine-protein kinase D3",
  "gene_symbol": "PRKD3",
  "term_id": "GO:0004674",
  "term_label": "protein serine/threonine kinase activity"
}